lymphocyte migration into lymphoid organs [GO:0097021] (biological process) Also known as: lymphocyte homing Definition: The movement of a lymphocyte within the lymphatic system into lymphoid organs such as lymph nodes, spleen or Peyer's patches, and its subsequent positioning within defined functional compartments such as sites of cell activation by antigen. Subtypes: lymphocyte migration into lymph node [GO:0097022] References: PMID:18379575 Sources: GOC:BHF, GOC:pr Relationships: is a type of lymphocyte migration [GO:0072676]